{
  "gene_symbol": "PRPSAP1",
  "gene": "UniProtKB:Q14558",
  "term_id": "GO:0030234",
  "gene_name": "Phosphoribosyl pyrophosphate synthase-associated protein 1",
  "term_label": "enzyme regulator activity"
}